{
  "gene_name": "ATP-dependent 6-phosphofructokinase, platelet type",
  "term_label": "fructose 6-phosphate metabolic process",
  "term_id": "GO:0006002",
  "gene": "UniProtKB:Q01813",
  "gene_symbol": "PFKP"
}